{
  "gene_name": "Transmembrane and coiled-coil domain-containing protein 5B",
  "gene_symbol": "TMCO5B",
  "term_label": "Unknown cellular component",
  "gene": "UniProtKB:A8MYB1",
  "term_id": "UNKNOWN:0003"
}